{
  "gene": "UniProtKB:Q9BQS2",
  "gene_name": "Synaptotagmin-15",
  "term_label": "exocytic vesicle",
  "term_id": "GO:0070382",
  "gene_symbol": "SYT15"
}